receptor-mediated endocytosis [GO:0006898] (biological process) Regulation: RO_0002211 by regulation of receptor-mediated endocytosis [GO:0048259]; positively regulated by GO:0048260; negatively regulated by negative regulation of receptor-mediated endocytosis [GO:0048261] Relationships: is a type of endocytosis [GO:0006897] Also known as: receptor mediated endocytosis Sources: GOC:mah, ISBN:0716731363 Definition: An endocytosis process in which cell surface receptors ensure specificity of transport. A specific receptor on the cell surface binds tightly to the extracellular macromolecule (the ligand) that it recognizes; the plasma-membrane region containing the receptor-ligand complex then undergoes endocytosis, forming a transport vesicle containing the receptor-ligand complex and excluding most other plasma-membrane proteins. Receptor-mediated endocytosis generally occurs via clathrin-coated pits and vesicles. Subtypes: GO:0019065, endocytic hemoglobin import into cell [GO:0020028], receptor internalization [GO:0031623], GO:0072583, receptor-mediated endocytosis involved in cholesterol transport [GO:0090118], endocytic iron import into cell [GO:0140298], GO:0160006